{
  "gene": "UniProtKB:Q9BZG1",
  "term_id": "GO:0043001",
  "gene_symbol": "RAB34",
  "term_label": "Golgi to plasma membrane protein transport",
  "gene_name": "Ras-related protein Rab-34"
}